superoxide dismutase copper chaperone complex [GO:1902694] (cellular component) Definition: A protein complex which is capable of superoxide dismutase copper chaperone activity. Relationships: is a type of metallochaperone complex [GO:1902695] Note: An example of this is CCS1 in Saccharomyces cerevisiae S288c (UniProt symbol P40202) in PMID:10426947. References: PMID:10426947 Sources: GOC:TermGenie, GOC:bhm, GO_REF:0000088